{
  "gene_symbol": "REEP3",
  "gene": "UniProtKB:Q6NUK4",
  "term_label": "endoplasmic reticulum tubular network",
  "gene_name": "Receptor expression-enhancing protein 3",
  "term_id": "GO:0071782"
}